{
  "term_id": "GO:0030198",
  "term_label": "extracellular matrix organization",
  "gene": "UniProtKB:Q14055",
  "gene_name": "Collagen alpha-2(IX) chain",
  "gene_symbol": "COL9A2"
}